{
  "gene_symbol": "HSPA4",
  "gene": "UniProtKB:P34932",
  "term_id": "GO:0005634",
  "gene_name": "Heat shock 70 kDa protein 4",
  "term_label": "nucleus"
}